galacturonate transmembrane transporter activity [GO:0015550] (MF) Relationships: is a type of carboxylic acid transmembrane transporter activity [GO:0046943]; is part of galacturonate transmembrane transport [GO:0015737] Sources: GOC:ai Definition: Enables the transfer of galacturonate from one side of a membrane to the other. Galacturonate is the uronic acid formally derived from galactose by oxidation of the hydroxymethylene group at C-6 to a carboxyl group.